{
  "gene_symbol": "S1PR2",
  "term_id": "GO:0003376",
  "gene_name": "Sphingosine 1-phosphate receptor 2",
  "term_label": "sphingosine-1-phosphate receptor signaling pathway",
  "gene": "UniProtKB:O95136"
}